{
  "gene_symbol": "ASPG",
  "term_id": "UNKNOWN:0002",
  "gene_name": "60 kDa lysophospholipase",
  "gene": "UniProtKB:Q86U10",
  "term_label": "Unknown biological process"
}